3-methylbutanal reductase (NADH) activity [GO:0052676] (molecular function) Also known as: 3-methylbutanal reductase (NAD) activity, 3-methylbutanol:NAD oxidoreductase activity, 3-methylbutyraldehyde reductase (NAD) activity, isoamyl alcohol oxidase (NAD) activity, 3-methylbutanol:NAD+ oxidoreductase activity Definition: Catalysis of the reaction: 3-methylbutanol + NAD+ = 3-methylbutanal + NADH + H+. 3-methylbutanal is also known as isovaleraldehyde. Sources: KEGG_REACTION:R05685, RHEA:18529 Relationships: is a type of alcohol dehydrogenase (NAD+) activity [GO:0004022]; is a type of 3-methylbutanal reductase [NAD(P)H] activity [GO:0046568]